{
  "gene_name": "Putative olfactory receptor 2B8",
  "term_label": "olfactory receptor activity",
  "term_id": "GO:0004984",
  "gene_symbol": "OR2B8",
  "gene": "UniProtKB:P59922"
}